regulation of transport across blood-brain barrier [GO:0150200] (biological process) References: PMID:29377008, PMID:30280653 Sources: GOC:aruk, GOC:bc Definition: Any process that modulates the frequency, rate or extent of transport across the blood-brain barrier. Subtypes: positive regulation of transport across blood-brain barrier [GO:0150201], negative regulation of transport across blood-brain barrier [GO:0150202], regulation of lipid transport across blood-brain barrier [GO:1903000] Relationships: is a type of regulation of system process [GO:0044057]; is a type of regulation of transport [GO:0051049]; is part of GO:0043114; regulates transport across blood-brain barrier [GO:0150104]